{
  "gene_symbol": "LAMB3",
  "gene_name": "Laminin subunit beta-3",
  "term_label": "extracellular space",
  "term_id": "GO:0005615",
  "gene": "UniProtKB:Q13751"
}